{
  "gene_symbol": "MCPH1",
  "gene": "UniProtKB:Q8NEM0",
  "term_label": "Unknown cellular component",
  "gene_name": "Microcephalin",
  "term_id": "UNKNOWN:0003"
}